{
  "gene": "UniProtKB:O95573",
  "gene_name": "Fatty acid CoA ligase Acsl3",
  "term_label": "long-chain fatty acid metabolic process",
  "term_id": "GO:0001676",
  "gene_symbol": "ACSL3"
}